{
  "gene_symbol": "NEUROD2",
  "term_label": "sensory organ development",
  "gene": "UniProtKB:Q15784",
  "gene_name": "Neurogenic differentiation factor 2",
  "term_id": "GO:0007423"
}